{
  "term_label": "ribosomal large subunit biogenesis",
  "gene_name": "Nucleophosmin",
  "gene_symbol": "NPM1",
  "gene": "UniProtKB:P06748",
  "term_id": "GO:0042273"
}